{
  "gene_symbol": "SUV39H2",
  "gene_name": "Histone-lysine N-methyltransferase SUV39H2",
  "term_label": "histone H3K9 methyltransferase activity",
  "gene": "UniProtKB:Q9H5I1",
  "term_id": "GO:0046974"
}